D-serine transmembrane transport [GO:0042942] (BP) Sources: GOC:jl, GOC:jsg, GOC:mah Relationships: is a type of amino acid transmembrane transport [GO:0003333]; is a type of serine transport [GO:0032329]; is_a GO:0042940; is a type of carboxylic acid transmembrane transport [GO:1905039] Definition: The process in which of D-serine, the D-enantiomer of 2-amino-3-hydroxypropanoic acid is transported across a lipid bilayer, from one side of a membrane to the other, by means of some agent such as a transporter or pore.